{
  "gene": "UniProtKB:Q8NC24",
  "gene_symbol": "RELL2",
  "term_label": "positive regulation of p38MAPK cascade",
  "gene_name": "RELT-like protein 2",
  "term_id": "GO:1900745"
}